{
  "gene": "UniProtKB:Q96DE0",
  "gene_symbol": "NUDT16",
  "term_id": "GO:1990174",
  "term_label": "phosphodiesterase decapping endonuclease activity",
  "gene_name": "U8 snoRNA-decapping enzyme"
}